{
  "gene_name": "Ubiquitin carboxyl-terminal hydrolase MINDY-1",
  "gene_symbol": "MINDY1",
  "term_label": "cysteine-type carboxypeptidase activity",
  "gene": "UniProtKB:Q8N5J2",
  "term_id": "GO:0016807"
}